{
  "gene_name": "Proline-rich protein 18",
  "term_id": "UNKNOWN:0002",
  "gene": "UniProtKB:Q8N4B5",
  "term_label": "Unknown biological process",
  "gene_symbol": "PRR18"
}